{
  "gene_symbol": "KLHDC4",
  "gene_name": "Kelch domain-containing protein 4",
  "gene": "UniProtKB:Q8TBB5",
  "term_label": "Unknown molecular function",
  "term_id": "UNKNOWN:0001"
}